{
  "gene_symbol": "CYGB",
  "gene": "UniProtKB:Q8WWM9",
  "term_id": "UNKNOWN:0002",
  "gene_name": "Cytoglobin",
  "term_label": "Unknown biological process"
}